{
  "gene_symbol": "PTK2",
  "term_id": "GO:0007173",
  "term_label": "epidermal growth factor receptor signaling pathway",
  "gene": "UniProtKB:Q05397",
  "gene_name": "Focal adhesion kinase 1"
}